{
  "gene_symbol": "UGT8",
  "gene_name": "2-hydroxyacylsphingosine 1-beta-galactosyltransferase",
  "gene": "UniProtKB:Q16880",
  "term_id": "GO:0005783",
  "term_label": "endoplasmic reticulum"
}